{
  "gene": "UniProtKB:P14555",
  "term_label": "calcium-dependent phospholipase A2 activity",
  "gene_name": "Phospholipase A2, membrane associated",
  "gene_symbol": "PLA2G2A",
  "term_id": "GO:0047498"
}